negative regulation of macrophage chemotaxis [GO:0010760] (biological process) Definition: Any process that decreases the rate, frequency or extent of macrophage chemotaxis. Macrophage chemotaxis is the movement of a macrophage in response to an external stimulus. Sources: GOC:BHF, GOC:dph, GOC:tb Relationships: is_a negative regulation of leukocyte chemotaxis [GO:0002689]; is a type of regulation of macrophage chemotaxis [GO:0010758]; is a type of negative regulation of macrophage migration [GO:1905522]; negatively regulates macrophage chemotaxis [GO:0048246]